{
  "term_label": "T cell activation involved in immune response",
  "gene_name": "Interferon alpha-5",
  "gene": "UniProtKB:P01569",
  "gene_symbol": "IFNA5",
  "term_id": "GO:0002286"
}